{
  "term_label": "peptide YY receptor activity",
  "gene_symbol": "NPY1R",
  "gene_name": "Neuropeptide Y receptor type 1",
  "gene": "UniProtKB:P25929",
  "term_id": "GO:0001601"
}